{
  "gene": "UniProtKB:Q9Y689",
  "term_id": "GO:1903292",
  "gene_symbol": "ARL5A",
  "gene_name": "ADP-ribosylation factor-like protein 5A",
  "term_label": "protein localization to Golgi membrane"
}